{
  "gene_name": "ARF GTPase-activating protein GIT1",
  "gene": "UniProtKB:Q9Y2X7",
  "term_id": "GO:0008277",
  "term_label": "regulation of G protein-coupled receptor signaling pathway",
  "gene_symbol": "GIT1"
}